DNA repair complex assembly [GO:0090735] (biological process) Definition: The aggregation, arrangement and bonding together of a set of components to form a DNA repair complex. Subtypes: GO:0000730, DNA recombinase mediator complex assembly [GO:1903871] References: PMID:27113759, PMID:27233470 Sources: GOC:pg Relationships: is a type of protein-containing complex assembly [GO:0065003]